retinol isomerase activity [GO:0050251] (molecular function) Relationships: is a type of cis-trans isomerase activity [GO:0016859] Sources: GOC:pde, RHEA:19141 Definition: Catalysis of the reaction: all-trans-retinol = 11-cis-retinol. Also known as: all-trans-retinol 11-cis-trans-isomerase activity, all-trans-retinol isomerase activity